{
  "gene_symbol": "IGKV1-27",
  "term_id": "GO:0006955",
  "gene": "UniProtKB:A0A075B6S5",
  "gene_name": "Immunoglobulin kappa variable 1-27",
  "term_label": "immune response"
}